{
  "term_id": "GO:0008017",
  "term_label": "microtubule binding",
  "gene_symbol": "MAP1A",
  "gene": "UniProtKB:P78559",
  "gene_name": "Microtubule-associated protein 1A"
}